CD8-positive, alpha-beta T cell extravasation [GO:0035697] (biological process) Subtypes: T-helper 1 cell extravasation [GO:0035687], CD8-positive, alpha-beta cytotoxic T cell extravasation [GO:0035698], T-helper 17 cell extravasation [GO:0035699] Regulation: regulated by regulation of CD8-positive, alpha-beta T cell extravasation [GO:2000449]; negatively regulated by GO:2000450; positively regulated by GO:2000451 Definition: The migration of a CD8-positive, alpha-beta T cell from the blood vessels into the surrounding tissue. Sources: CL:0000625, GOC:BHF Relationships: is a type of T cell extravasation [GO:0072683]